{
  "gene": "UniProtKB:Q495M9",
  "gene_name": "pre-mRNA splicing regulator USH1G",
  "term_id": "UNKNOWN:0001",
  "term_label": "Unknown molecular function",
  "gene_symbol": "USH1G"
}